{
  "term_label": "negative regulation of transcription by RNA polymerase II",
  "gene": "UniProtKB:P10827",
  "gene_name": "Thyroid hormone receptor alpha",
  "gene_symbol": "THRA",
  "term_id": "GO:0000122"
}